{
  "gene_name": "RNA-binding protein Nova-2",
  "term_label": "nucleus",
  "term_id": "GO:0005634",
  "gene_symbol": "NOVA2",
  "gene": "UniProtKB:Q9UNW9"
}